{
  "term_label": "Unknown cellular component",
  "gene_name": "T cell receptor alpha variable 26-2",
  "gene_symbol": "TRAV26-2",
  "term_id": "UNKNOWN:0003",
  "gene": "UniProtKB:A0A0B4J265"
}